{
  "gene_symbol": "VBP1",
  "gene_name": "Prefoldin subunit 3",
  "gene": "UniProtKB:P61758",
  "term_id": "GO:0016272",
  "term_label": "prefoldin complex"
}